{
  "gene_name": "Checkpoint protein HUS1B",
  "term_label": "mitotic intra-S DNA damage checkpoint signaling",
  "gene": "UniProtKB:Q8NHY5",
  "gene_symbol": "HUS1B",
  "term_id": "GO:0031573"
}